glycine oxidase activity [GO:0043799] (molecular function) Also known as: glycine:oxygen oxidoreductase (deaminating) Sources: EC:1.4.3.19 Definition: Catalysis of the reactions: (1) glycine + H2O + O2 = glyoxylate + NH3 + hydrogen peroxide; (2) D-alanine + H2O + O2 = pyruvate + NH3 + hydrogen peroxide; (3) sarcosine + H2O + O2 = glyoxylate + methylamine + hydrogen peroxide; (4) N-ethylglycine + H2O + O2 = glyoxylate + ethylamine + hydrogen peroxide. Relationships: is a type of aliphatic amine oxidase activity [GO:0052595]